{
  "gene_symbol": "BPY2",
  "term_label": "nucleus",
  "term_id": "GO:0005634",
  "gene": "UniProtKB:O14599",
  "gene_name": "Testis-specific basic protein Y 2"
}